{
  "term_id": "GO:0045182",
  "gene_name": "Fragile X messenger ribonucleoprotein 1",
  "gene": "UniProtKB:Q06787",
  "gene_symbol": "FMR1",
  "term_label": "translation regulator activity"
}